{
  "gene_name": "Ergosterol biosynthetic protein 28 homolog",
  "gene_symbol": "ERG28",
  "term_label": "Unknown biological process",
  "gene": "UniProtKB:Q9UKR5",
  "term_id": "UNKNOWN:0002"
}